{
  "gene": "UniProtKB:Q70Z44",
  "term_label": "serotonin-gated monoatomic cation channel activity",
  "gene_symbol": "HTR3D",
  "term_id": "GO:0022850",
  "gene_name": "5-hydroxytryptamine receptor 3D"
}